{
  "gene_symbol": "HAPLN1",
  "gene": "UniProtKB:P10915",
  "term_label": "central nervous system development",
  "gene_name": "Hyaluronan and proteoglycan link protein 1",
  "term_id": "GO:0007417"
}